{
  "gene": "UniProtKB:Q9HD20",
  "gene_name": "Endoplasmic reticulum transmembrane helix translocase",
  "term_id": "GO:0006874",
  "gene_symbol": "ATP13A1",
  "term_label": "intracellular calcium ion homeostasis"
}